{
  "gene_name": "Deuterosome assembly protein 1",
  "term_label": "centriole replication",
  "term_id": "GO:0007099",
  "gene_symbol": "DEUP1",
  "gene": "UniProtKB:Q05D60"
}